nuclear chromosome [GO:0000228] (cellular component) Definition: A chromosome that encodes the nuclear genome and is found in the nucleus of a eukaryotic cell during the cell cycle phases when the nucleus is intact. Subtypes: condensed nuclear chromosome [GO:0000794], Barr body [GO:0001740] Relationships: is a type of chromosome [GO:0005694]; is part of nuclear lumen [GO:0031981] Also known as: nuclear interphase chromosome Sources: GOC:dph, GOC:mah